{
  "term_id": "GO:0000976",
  "term_label": "transcription cis-regulatory region binding",
  "gene": "UniProtKB:Q86WZ6",
  "gene_name": "Zinc finger protein 227",
  "gene_symbol": "ZNF227"
}